{
  "term_label": "cytoplasm",
  "gene_name": "SH3 and PX domain-containing protein 2B",
  "gene_symbol": "SH3PXD2B",
  "gene": "UniProtKB:A1X283",
  "term_id": "GO:0005737"
}